{
  "gene_symbol": "STOX2",
  "gene_name": "Storkhead-box protein 2",
  "term_id": "GO:0005737",
  "gene": "UniProtKB:Q9P2F5",
  "term_label": "cytoplasm"
}